{
  "term_label": "ribosomal small subunit assembly",
  "term_id": "GO:0000028",
  "gene_name": "Ribosomal RNA-processing protein 7 homolog A",
  "gene": "UniProtKB:Q9Y3A4",
  "gene_symbol": "RRP7A"
}